{
  "term_label": "double-strand break repair",
  "gene_symbol": "APLF",
  "gene_name": "Aprataxin and PNK-like factor",
  "gene": "UniProtKB:Q8IW19",
  "term_id": "GO:0006302"
}